{
  "term_label": "Unknown cellular component",
  "gene_symbol": "METTL5",
  "gene_name": "rRNA N6-adenosine-methyltransferase METTL5",
  "gene": "UniProtKB:Q9NRN9",
  "term_id": "UNKNOWN:0003"
}